{
  "term_id": "GO:0005634",
  "gene_symbol": "OGG1",
  "gene_name": "N-glycosylase_DNA lyase",
  "term_label": "nucleus",
  "gene": "UniProtKB:O15527"
}